{
  "gene_name": "Protein YIF1B",
  "gene": "UniProtKB:Q5BJH7",
  "term_label": "endoplasmic reticulum-Golgi intermediate compartment",
  "term_id": "GO:0005793",
  "gene_symbol": "YIF1B"
}